viral capsid secondary envelopment [GO:0046745] (biological process) Definition: The process in which a capsid acquires another membrane envelope, subsequent to acquiring an initial membrane envelope. References: PMID:11533156 Sources: ISBN:0072370319, ISBN:0781718325 Also known as: outer nuclear membrane viral budding during viral capsid re-envelopment, viral budding from ER membrane by viral capsid re-envelopment, viral budding from Golgi membrane by viral capsid re-envelopment, viral budding from inner nuclear membrane by viral capsid re-envelopment, viral budding from nuclear membrane by viral capsid re-envelopment, viral budding from outer nuclear membrane by viral capsid re-envelopment, viral budding from outer nuclear membrane during viral capsid re-envelopment, viral budding from plasma membrane by viral capsid re-envelopment, virus budding from ER membrane by viral capsid re-envelopment, virus budding from Golgi membrane by viral capsid re-envelopment, virus budding from inner nuclear membrane by viral capsid re-envelopment, virus budding from nuclear membrane by viral capsid re-envelopment, virus budding from outer nuclear membrane by viral capsid re-envelopment, ER membrane viral budding during viral capsid re-envelopment, Golgi membrane viral budding during viral capsid re-envelopment, endoplasmic reticulum membrane viral budding during viral capsid re-envelopment, inner nuclear membrane viral budding during viral capsid re-envelopment, nuclear membrane viral budding during viral capsid re-envelopment, plasma membrane viral budding during viral capsid re-envelopment, viral budding from ER membrane during viral capsid re-envelopment, viral budding from Golgi membrane during viral capsid re-envelopment, viral budding from inner nuclear membrane during viral capsid re-envelopment, viral budding from nuclear membrane during viral capsid re-envelopment, viral budding from plasma membrane during viral capsid re-envelopment, viral capsid re-envelopment, virus budding from ER membrane during viral capsid re-envelopment, virus budding from Golgi membrane during viral capsid re-envelopment, virus budding from inner nuclear membrane during viral capsid re-envelopment, virus budding from nuclear membrane during viral capsid re-envelopment, virus budding from outer nuclear membrane during viral capsid re-envelopment, virus budding from plasma membrane during viral capsid re-envelopment Relationships: is a type of viral process [GO:0016032]